{
  "gene": "UniProtKB:Q9Y5I4",
  "gene_name": "Protocadherin alpha-C2",
  "gene_symbol": "PCDHAC2",
  "term_id": "GO:0007155",
  "term_label": "cell adhesion"
}